{
  "gene_symbol": "RYBP",
  "gene": "UniProtKB:Q8N488",
  "term_label": "DNA binding",
  "gene_name": "RING1 and YY1-binding protein",
  "term_id": "GO:0003677"
}